melatonin catabolic process [GO:0042442] (biological process) Definition: The chemical reactions and pathways resulting in the breakdown of melatonin (N-acetyl-5-methoxytryptamine). Sources: GOC:jl Also known as: melatonin breakdown, melatonin catabolism, melatonin degradation Relationships: is a type of melatonin metabolic process [GO:0030186]; is a type of indole-containing compound catabolic process [GO:0042436]; is a type of hormone catabolic process [GO:0042447]